{
  "gene_name": "Angiopoietin-4",
  "term_id": "GO:0030971",
  "gene": "UniProtKB:Q9Y264",
  "gene_symbol": "ANGPT4",
  "term_label": "receptor tyrosine kinase binding"
}